{
  "term_id": "GO:0017071",
  "gene_symbol": "CNGA3",
  "term_label": "intracellular cyclic nucleotide activated cation channel complex",
  "gene_name": "Cyclic nucleotide-gated cation channel alpha-3",
  "gene": "UniProtKB:Q16281"
}